UDP-glucuronate biosynthetic process [GO:0006065] (biological process) Also known as: UDP-glucuronate anabolism, UDP-glucuronate biosynthesis, UDP-glucuronate formation, UDP-glucuronate synthesis Relationships: is a type of nucleotide-sugar biosynthetic process [GO:0009226]; is a type of carboxylic acid biosynthetic process [GO:0046394]; is a type of UDP-glucuronate metabolic process [GO:0046398] Sources: GOC:ai Definition: The chemical reactions and pathways resulting in the formation of UDP-glucuronate, a substance composed of glucuronic acid in glycosidic linkage with uridine diphosphate.